equatorial microtubule organizing center assembly [GO:1904185] (biological process) Also known as: EMTOC assembly, EMTOC formation, equatorial microtubule organising centre assembly, equatorial microtubule organising centre formation, equatorial microtubule organizing center formation Definition: The aggregation, arrangement and bonding together of a set of components to form an equatorial microtubule organizing center. References: PMID:15004232 Sources: GOC:TermGenie, GO_REF:0000079 Relationships: is a type of GO:0022607; is a type of GO:0031023